{
  "gene": "UniProtKB:Q8NI35",
  "term_id": "GO:0005886",
  "gene_symbol": "PATJ",
  "gene_name": "InaD-like protein",
  "term_label": "plasma membrane"
}